histone H3K56 methyltransferase activity [GO:0140759] (molecular function) References: PMID:23451023, PMID:28743002 Relationships: is a type of protein-lysine N-methyltransferase activity [GO:0016279]; is a type of histone H3 methyltransferase activity [GO:0140938] Note: Comment: Note that the residue position corresponds to the canonical human H3 histone (UniProtKB:P84243); this residue is conserved across all eukaryotes. Residue 1 is the first residue following removal of the initiating Methionine (Met). Note that each histone is encoded by multiple genes, and sequences may vary across different genes within an organism. Definition: Catalysis of the reaction: S-adenosyl-L-methionine + histone H3 L-lysine (position 56) = S-adenosyl-L-homocysteine + histone H3 N6-methyl-L-lysine (position 56). This reaction is the addition of a methyl group to the lysine residue at position 56 of the histone H3 protein. Also known as: histone H3K56 methylase activity, histone lysine N-methyltransferase activity (H3-K56 specific), histone methyltransferase activity (H3-K56 specific), histone-H3K56 methyltransferase activity